{
  "gene": "UniProtKB:Q96AP4",
  "term_label": "regulation of DNA-templated transcription",
  "gene_name": "Zinc finger-containing ubiquitin peptidase 1",
  "gene_symbol": "ZUP1",
  "term_id": "GO:0006355"
}